{
  "gene_symbol": "DNMT3B",
  "gene_name": "DNA (cytosine-5)-methyltransferase 3B",
  "term_label": "DNA (cytosine-5-)-methyltransferase activity, acting on CpG substrates",
  "gene": "UniProtKB:Q9UBC3",
  "term_id": "GO:0051718"
}